{
  "gene_name": "Putative uncharacterized protein encoded by LINC01356",
  "gene": "UniProtKB:Q8N9X3",
  "gene_symbol": "LINC01356",
  "term_label": "Unknown molecular function",
  "term_id": "UNKNOWN:0001"
}